{
  "term_id": "GO:0006357",
  "term_label": "regulation of transcription by RNA polymerase II",
  "gene": "UniProtKB:A6NHT5",
  "gene_symbol": "HMX3",
  "gene_name": "Homeobox protein HMX3"
}